{
  "gene_name": "5-methylcytosine rRNA methyltransferase NSUN4",
  "gene_symbol": "NSUN4",
  "term_label": "Unknown cellular component",
  "term_id": "UNKNOWN:0003",
  "gene": "UniProtKB:Q96CB9"
}